{
  "gene_name": "Amyloid-beta A4 precursor protein-binding family B member 3",
  "gene_symbol": "APBB3",
  "term_label": "amyloid-beta binding",
  "term_id": "GO:0001540",
  "gene": "UniProtKB:O95704"
}